geraniol 10-hydroxylase activity [GO:0102811] (molecular function) Definition: Catalysis of the reaction: geraniol + O2 + NADPH + H+ = (6E)-8-hydroxygeraniol + NADP + H2O. Relationships: is a type of GO:0016709 Sources: EC:1.14.14.83, GOC:pz